{
  "term_label": "cytoplasm",
  "gene": "UniProtKB:O00311",
  "gene_symbol": "CDC7",
  "gene_name": "Cell division cycle 7-related protein kinase",
  "term_id": "GO:0005737"
}